{
  "gene_name": "Adenosine 5'-monophosphoramidase HINT1",
  "term_label": "nucleus",
  "gene_symbol": "HINT1",
  "term_id": "GO:0005634",
  "gene": "UniProtKB:P49773"
}